{
  "term_id": "GO:0030667",
  "gene_symbol": "SCG3",
  "term_label": "secretory granule membrane",
  "gene": "UniProtKB:Q8WXD2",
  "gene_name": "Secretogranin-3"
}